{
  "term_label": "cytoplasm",
  "gene_symbol": "AGBL3",
  "gene": "UniProtKB:Q8NEM8",
  "term_id": "GO:0005737",
  "gene_name": "Cytosolic carboxypeptidase 3"
}